{
  "term_label": "fumarate transmembrane transporter activity",
  "gene": "UniProtKB:Q13183",
  "gene_symbol": "SLC13A2",
  "term_id": "GO:0015138",
  "gene_name": "Solute carrier family 13 member 2"
}